{
  "term_id": "UNKNOWN:0001",
  "gene": "UniProtKB:Q6P499",
  "term_label": "Unknown molecular function",
  "gene_symbol": "NIPAL3",
  "gene_name": "NIPA-like protein 3"
}